{
  "term_label": "glutaminyl-tRNA aminoacylation",
  "gene": "UniProtKB:P47897",
  "gene_name": "Glutamine--tRNA ligase",
  "term_id": "GO:0006425",
  "gene_symbol": "QARS1"
}